{
  "gene_name": "Zinc finger protein 862",
  "term_label": "Unknown cellular component",
  "gene": "UniProtKB:O60290",
  "term_id": "UNKNOWN:0003",
  "gene_symbol": "ZNF862"
}